{
  "gene_name": "Rab11 family-interacting protein 4",
  "gene_symbol": "RAB11FIP4",
  "gene": "UniProtKB:Q86YS3",
  "term_id": "GO:0030496",
  "term_label": "midbody"
}